{
  "gene": "UniProtKB:P52732",
  "gene_symbol": "KIF11",
  "term_id": "GO:0008574",
  "gene_name": "Kinesin-like protein KIF11",
  "term_label": "plus-end-directed microtubule motor activity"
}